{
  "gene_name": "Kinesin-like protein KIF28P",
  "gene": "UniProtKB:B7ZC32",
  "gene_symbol": "KIF28P",
  "term_label": "microtubule",
  "term_id": "GO:0005874"
}